regulation of seed growth [GO:0080113] (biological process) Relationships: is_a GO:0048638; regulates seed growth [GO:0080112] References: PMID:19141706 Definition: Any process that modulates the frequency, rate or extent of growth of the seed of an plant. Also known as: regulation of seed size